{
  "term_label": "receptor complex",
  "term_id": "GO:0043235",
  "gene_name": "Ephrin type-B receptor 4",
  "gene_symbol": "EPHB4",
  "gene": "UniProtKB:P54760"
}